{
  "term_id": "UNKNOWN:0003",
  "gene_name": "Matrix metalloproteinase-21",
  "gene": "UniProtKB:Q8N119",
  "gene_symbol": "MMP21",
  "term_label": "Unknown cellular component"
}